negative regulation of B cell chemotaxis [GO:2000550] (biological process) Sources: GOC:obol Relationships: is a type of negative regulation of lymphocyte chemotaxis [GO:1901624]; is a type of regulation of B cell chemotaxis [GO:2000537]; negatively regulates B cell chemotaxis [GO:0035754] Definition: Any process that stops, prevents or reduces the frequency, rate or extent of B cell chemotaxis.